{
  "term_id": "GO:0071565",
  "gene": "UniProtKB:Q8TAQ2",
  "gene_name": "SWI_SNF complex subunit SMARCC2",
  "gene_symbol": "SMARCC2",
  "term_label": "nBAF complex"
}